{
  "term_id": "GO:0005739",
  "gene_symbol": "GPAT2",
  "gene": "UniProtKB:Q6NUI2",
  "gene_name": "Glycerol-3-phosphate acyltransferase 2, mitochondrial",
  "term_label": "mitochondrion"
}